{
  "gene_name": "Cysteine-rich DPF motif domain-containing protein 1",
  "gene": "UniProtKB:Q6NVV7",
  "term_id": "UNKNOWN:0003",
  "term_label": "Unknown cellular component",
  "gene_symbol": "CDPF1"
}